{
  "gene": "UniProtKB:Q9UKA8",
  "gene_name": "Calcipressin-3",
  "term_id": "GO:0019722",
  "gene_symbol": "RCAN3",
  "term_label": "calcium-mediated signaling"
}